{
  "term_id": "GO:0006897",
  "gene": "UniProtKB:O75146",
  "term_label": "endocytosis",
  "gene_symbol": "HIP1R",
  "gene_name": "Huntingtin-interacting protein 1-related protein"
}